{
  "gene_name": "Acid-sensing ion channel 5",
  "term_id": "GO:0035725",
  "gene_symbol": "ASIC5",
  "gene": "UniProtKB:Q9NY37",
  "term_label": "sodium ion transmembrane transport"
}